{
  "term_label": "cardiac muscle tissue development",
  "gene_name": "Gamma-sarcoglycan",
  "gene_symbol": "SGCG",
  "gene": "UniProtKB:Q13326",
  "term_id": "GO:0048738"
}